{
  "gene_symbol": "RNF144B",
  "gene_name": "E3 ubiquitin-protein ligase RNF144B",
  "gene": "UniProtKB:Q7Z419",
  "term_label": "ubiquitin conjugating enzyme binding",
  "term_id": "GO:0031624"
}